{
  "term_label": "Unknown molecular function",
  "term_id": "UNKNOWN:0001",
  "gene_symbol": "TRMT2A",
  "gene": "UniProtKB:Q8IZ69",
  "gene_name": "tRNA (uracil-5-)-methyltransferase homolog A"
}